{
  "term_id": "GO:0043065",
  "term_label": "positive regulation of apoptotic process",
  "gene_symbol": "BCL2A1",
  "gene": "UniProtKB:Q16548",
  "gene_name": "Bcl-2-related protein A1"
}